{
  "gene": "UniProtKB:Q16585",
  "gene_name": "Beta-sarcoglycan",
  "term_id": "UNKNOWN:0002",
  "term_label": "Unknown biological process",
  "gene_symbol": "SGCB"
}